{
  "gene": "UniProtKB:Q92551",
  "term_label": "inositol hexakisphosphate kinase activity",
  "gene_symbol": "IP6K1",
  "term_id": "GO:0000828",
  "gene_name": "Inositol hexakisphosphate kinase 1"
}